{
  "gene": "UniProtKB:P49368",
  "gene_symbol": "CCT3",
  "gene_name": "T-complex protein 1 subunit gamma",
  "term_label": "protein folding",
  "term_id": "GO:0006457"
}